{
  "gene_name": "Nitric oxide synthase 1",
  "term_label": "nitric oxide biosynthetic process",
  "gene_symbol": "NOS1",
  "gene": "UniProtKB:P29475",
  "term_id": "GO:0006809"
}